cellular response to steroid hormone stimulus [GO:0071383] (biological process) Relationships: is a type of GO:0032870; is a type of GO:0048545; is a type of GO:0071396 Subtypes: cellular response to corticosteroid stimulus [GO:0071384], cellular response to progesterone stimulus [GO:0071393] Sources: GOC:mah Definition: Any process that results in a change in state or activity of a cell (in terms of movement, secretion, enzyme production, gene expression, etc.) as a result of a steroid hormone stimulus.